{
  "term_label": "polyubiquitin modification-dependent protein binding",
  "gene": "UniProtKB:Q96S82",
  "gene_symbol": "UBL7",
  "gene_name": "Ubiquitin-like protein 7",
  "term_id": "GO:0031593"
}